{
  "gene_symbol": "RYR2",
  "gene": "UniProtKB:Q92736",
  "gene_name": "Ryanodine receptor 2",
  "term_id": "GO:0042383",
  "term_label": "sarcolemma"
}